{
  "gene": "UniProtKB:A6NJ46",
  "gene_symbol": "NKX6-3",
  "term_id": "GO:0005634",
  "gene_name": "Homeobox protein Nkx-6.3",
  "term_label": "nucleus"
}